positive regulation of translational fidelity [GO:0045903] (biological process) Relationships: is a type of regulation of translational fidelity [GO:0006450]; is a type of GO:0045727 Also known as: up regulation of translational fidelity, up-regulation of translational fidelity, upregulation of translational fidelity, activation of translational fidelity, stimulation of translational fidelity Sources: GOC:dph, GOC:tb Definition: Any process that increases the ability of the translational apparatus to interpret the genetic code.